nuclear protein-containing complex [GO:0140513] (cellular component) Sources: GOC:pg Subtypes: nucleotide-excision repair complex [GO:0000109], histone deacetylase complex [GO:0000118], RNA polymerase I transcription regulator complex [GO:0000120], nuclear ubiquitin ligase complex [GO:0000152], GO:0000176, GO:0000214, GO:0000346, THO complex [GO:0000347], RNA polymerase IV complex [GO:0000418], RNA polymerase V complex [GO:0000419], GO:0000783, COMA complex [GO:0000817], GO:0002111, 5-lipoxygenase complex [GO:0002180], GO:0005643, GO:0005655, nuclear pre-replicative complex [GO:0005656], DNA replication factor A complex [GO:0005662], nuclear origin of replication recognition complex [GO:0005664], RNA polymerase III complex [GO:0005666], chromatin silencing complex [GO:0005677], spliceosomal complex [GO:0005681], telomerase holoenzyme complex [GO:0005697], RNA polymerase I complex [GO:0005736], GO:0005849, DNA-dependent protein kinase-DNA ligase 4 complex [GO:0005958], transcription elongation factor complex [GO:0008023], COP9 signalosome [GO:0008180], GO:0008622, mediator complex [GO:0016592], GO:0019908, small nuclear ribonucleoprotein complex [GO:0030532], Noc complex [GO:0030689], Mre11 complex [GO:0030870], apolipoprotein B mRNA editing enzyme complex [GO:0030895], checkpoint clamp complex [GO:0030896], GO:0030958, nuclear pore outer ring [GO:0031080], DNA replication preinitiation complex [GO:0031261], GO:0031298, GO:0031380, Ctf18 RFC-like complex [GO:0031390], GO:0031429, Dbf4-dependent protein kinase complex [GO:0031431], GO:0031499, SUMO activating enzyme complex [GO:0031510], CBF3 complex [GO:0031518], GO:0031519, Myb complex [GO:0031523], mRNA capping enzyme complex [GO:0031533], nuclear proteasome complex [GO:0031595], GO:0031598, GO:0031601, nuclear proteasome core complex, alpha-subunit complex [GO:0031604], GO:0031607, nuclear proteasome regulatory particle, base subcomplex [GO:0031610], nuclear proteasome regulatory particle, lid subcomplex [GO:0031613], GO:0032039, small-subunit processome [GO:0032040], SMC loading complex [GO:0032116], GO:0032301, MutSbeta complex [GO:0032302], GO:0032389, MutLbeta complex [GO:0032390], CURI complex [GO:0032545], Swi5-Sfr1 complex [GO:0032798], GO:0032806, DNA ligase IV complex [GO:0032807], Rad51B-Rad51C-Rad51D-XRCC2 complex [GO:0033063], XRCC2-RAD51D complex [GO:0033064], Rad51C-XRCC3 complex [GO:0033065], GO:0033066, GO:0033167, DNA helicase A complex [GO:0033203], Slx1-Slx4 complex [GO:0033557], mitotic checkpoint complex [GO:0033597], Mei2 nuclear dot complex [GO:0033620], Tor2-Mei2-Ste11 complex [GO:0034064], Pwp2p-containing subcomplex of 90S preribosome [GO:0034388], t-UTP complex [GO:0034455], UTP-C complex [GO:0034456], GO:0034457, GO:0034692, nuclear aryl hydrocarbon receptor complex [GO:0034753], Swi5-Swi2 complex [GO:0034974], PDX1-PBX1b-MRG1 complex [GO:0034978], GO:0034980, GO:0034981, RCAF complex [GO:0035059], histone methyltransferase complex [GO:0035097], exon-exon junction complex [GO:0035145], GO:0035808, histone H3-K14 acetyltransferase complex [GO:0036409], nuclear RNA export factor complex [GO:0042272], DASH complex [GO:0042729], Fanconi anaemia nuclear complex [GO:0043240], GO:0043564, nuclear DNA replication factor C complex [GO:0043599], nuclear replisome [GO:0043601], delta DNA polymerase complex [GO:0043625], PCNA complex [GO:0043626], DNA polymerase III, proofreading complex [GO:0043845], DNA polymerase III, clamp loader complex [GO:0043846], DNA polymerase III, clamp loader chi/psi subcomplex [GO:0043847], nuclear pore inner ring [GO:0044611], nuclear pore linkers [GO:0044612], nuclear pore central transport channel [GO:0044613], nuclear pore cytoplasmic filaments [GO:0044614], GO:0044615, DNA polymerase III, core complex [GO:0044776], dosage compensation complex [GO:0046536], Lid2 complex [GO:0048189], nuclear DNA-directed RNA polymerase complex [GO:0055029], CENP-T-W-S-X complex [GO:0061838], LinE complex [GO:0062119], MutSgamma complex [GO:0062128], nuclear exosome targeting complex [GO:0062141], Smp focus [GO:0062238], GO:0070274, ATR-ATRIP complex [GO:0070310], RGS6-DNMT1-DMAP1 complex [GO:0070313], GO:0070353, GATA2-TAL1-TCF3-Lmo2 complex [GO:0070354], GO:0070390, DNA-dependent protein kinase complex [GO:0070418], DNA ligase III-XRCC1 complex [GO:0070421], RC-1 DNA recombination complex [GO:0070467], CAK-ERCC2 complex [GO:0070516], DNA replication factor C core complex [GO:0070517], BRCA1-A complex [GO:0070531], BRCA1-B complex [GO:0070532], BRCA1-C complex [GO:0070533], GO:0070545, BRISC complex [GO:0070552], PCNA-p21 complex [GO:0070557], SWI/SNF superfamily-type complex [GO:0070603], GO:0070693, nuclear pore transmembrane ring [GO:0070762], BRCA1-Rad51 complex [GO:0070767], SOSS complex [GO:0070876], GO:0070877, GO:0071159, GO:0071175, MAML2-RBP-Jkappa-ICN2 complex [GO:0071176], MAML2-RBP-Jkappa-ICN3 complex [GO:0071177], MAML2-RBP-Jkappa-ICN4 complex [GO:0071178], MAML3-RBP-Jkappa-ICN1 complex [GO:0071179], MAML3-RBP-Jkappa-ICN2 complex [GO:0071180], MAML3-RBP-Jkappa-ICN3 complex [GO:0071181], GO:0071182, histone pre-mRNA 3'end processing complex [GO:0071204], catenin-TCF7L2 complex [GO:0071664], DUBm complex [GO:0071819], FANCM-MHF complex [GO:0071821], box H/ACA scaRNP complex [GO:0072589], U2AF complex [GO:0089701], GO:0090570, RNA polymerase II transcription repressor complex [GO:0090571], RNA polymerase III transcription repressor complex [GO:0090572], GO:0090573, GO:0090574, RNA polymerase II transcription regulator complex [GO:0090575], box H/ACA telomerase RNP complex [GO:0090661], CENP-A recruiting complex [GO:0098654], synapsis initiation complex [GO:0106069], nuclear membrane protein complex [GO:0106083], RNA polymerase II termination complex [GO:0110103], INTAC complex [GO:0160232], mitotic checkpoint complex, CDC20-MAD2 subcomplex [GO:1990333], activated SUMO-E1 ligase complex [GO:1990354], nucleosome disassembly/reassembly complex [GO:1990453], Rhino-Deadlock-Cutoff Complex [GO:1990469], GO:1990477, Cry-Per complex [GO:1990512], GO:1990622, survivin complex [GO:1990713], GO:1990862 Definition: A stable assembly of two or more macromolecules, i.e. proteins, nucleic acids, carbohydrates or lipids, in which at least one component is a protein and the constituent parts function together in the nucleus. Also known as: nuclear complex Relationships: is a type of protein-containing complex [GO:0032991]; is part of nucleus [GO:0005634]